negative regulation of fat cell apoptotic process [GO:1904650] (biological process) References: PMID:17024416 Sources: GOC:TermGenie, GO_REF:0000058 Definition: Any process that stops, prevents or reduces the frequency, rate or extent of fat cell apoptotic process. Relationships: is a type of negative regulation of apoptotic process [GO:0043066]; is a type of regulation of fat cell apoptotic process [GO:1904649]; negatively regulates GO:1904606 Also known as: down regulation of adipocyte apoptotic process, down regulation of adipose cell apoptotic process, down regulation of fat cell apoptotic process, down-regulation of adipocyte apoptotic process, down-regulation of adipose cell apoptotic process, down-regulation of fat cell apoptotic process, downregulation of adipocyte apoptotic process, downregulation of adipose cell apoptotic process, downregulation of fat cell apoptotic process, negative regulation of adipocyte apoptotic process, negative regulation of adipose cell apoptotic process, down regulation of adipocyte apoptosis, down regulation of adipose cell apoptosis, down regulation of fat cell apoptosis, down-regulation of adipocyte apoptosis, down-regulation of adipose cell apoptosis, down-regulation of fat cell apoptosis, downregulation of adipocyte apoptosis, downregulation of adipose cell apoptosis, downregulation of fat cell apoptosis, inhibition of adipocyte apoptosis, inhibition of adipocyte apoptotic process, inhibition of adipose cell apoptosis, inhibition of adipose cell apoptotic process, inhibition of fat cell apoptosis, inhibition of fat cell apoptotic process, negative regulation of adipocyte apoptosis, negative regulation of adipose cell apoptosis, negative regulation of fat cell apoptosis